negative regulation of chemokine production [GO:0032682] (biological process) Sources: GOC:mah Definition: Any process that stops, prevents, or reduces the frequency, rate, or extent of chemokine production. Subtypes: GO:0032684, negative regulation of chemokine (C-X-C motif) ligand 9 production [GO:0035395], negative regulation of chemokine (C-C motif) ligand 6 production [GO:0035532], negative regulation of monocyte chemotactic protein-1 production [GO:0071638], negative regulation of macrophage inflammatory protein 1 alpha production [GO:0071641], GO:0071644, negative regulation of macrophage inflammatory protein-1 gamma production [GO:0071647], GO:0071650, GO:0071653, GO:0071659, negative regulation of chemokine (C-C motif) ligand 20 production [GO:1903885], GO:2000339, negative regulation of chemokine (C-X-C motif) ligand 2 production [GO:2000342] Relationships: is_a negative regulation of cytokine production [GO:0001818]; is a type of regulation of chemokine production [GO:0032642]; negatively regulates chemokine production [GO:0032602] Also known as: down regulation of chemokine production, down-regulation of chemokine production, downregulation of chemokine production, inhibition of chemokine production, negative regulation of chemokine biosynthetic process, negative regulation of chemokine secretion